D-alanine biosynthetic process [GO:0030632] (biological process) Sources: GOC:jsg, GOC:mah Relationships: is_a GO:0006523; is_a D-alanine metabolic process [GO:0046436]; is a type of D-amino acid biosynthetic process [GO:0046437] Also known as: D-alanine anabolism, D-alanine biosynthesis, D-alanine formation, D-alanine synthesis Definition: The chemical reactions and pathways resulting in the formation of D-alanine, the D-enantiomer of the amino acid alanine, i.e (2R)-2-aminopropanoic acid.